{
  "gene_symbol": "HTR3B",
  "gene": "UniProtKB:O95264",
  "term_id": "GO:0034220",
  "gene_name": "5-hydroxytryptamine receptor 3B",
  "term_label": "monoatomic ion transmembrane transport"
}